{
  "term_id": "GO:0072657",
  "gene": "UniProtKB:P30419",
  "gene_name": "Glycylpeptide N-tetradecanoyltransferase 1",
  "term_label": "protein localization to membrane",
  "gene_symbol": "NMT1"
}